{
  "term_id": "GO:0005525",
  "gene_symbol": "RAB11A",
  "gene": "UniProtKB:P62491",
  "term_label": "GTP binding",
  "gene_name": "Ras-related protein Rab-11A"
}